{
  "gene": "UniProtKB:Q9NPG2",
  "term_label": "Unknown cellular component",
  "gene_symbol": "NGB",
  "gene_name": "Neuroglobin",
  "term_id": "UNKNOWN:0003"
}